{
  "gene_symbol": "PIK3AP1",
  "gene_name": "Phosphoinositide 3-kinase adapter protein 1",
  "gene": "UniProtKB:Q6ZUJ8",
  "term_id": "GO:0005829",
  "term_label": "cytosol"
}